shamixanthone biosynthetic process [GO:1900793] (biological process) Definition: The chemical reactions and pathways resulting in the formation of shamixanthone. Sources: GOC:TermGenie, GOC:di Also known as: shamixanthone anabolism, shamixanthone biosynthesis, shamixanthone formation, shamixanthone synthesis Relationships: is a type of ketone biosynthetic process [GO:0042181]; is a type of secondary metabolite biosynthetic process [GO:0044550]; is a type of phenol-containing compound biosynthetic process [GO:0046189]